{
  "term_label": "P-body",
  "gene_name": "Protein PAT1 homolog 2",
  "gene_symbol": "PATL2",
  "term_id": "GO:0000932",
  "gene": "UniProtKB:C9JE40"
}